{
  "term_id": "GO:0019706",
  "gene": "UniProtKB:Q5W0Z9",
  "gene_name": "Palmitoyltransferase ZDHHC20",
  "gene_symbol": "ZDHHC20",
  "term_label": "protein-cysteine S-palmitoyltransferase activity"
}